{
  "term_label": "response to toxic substance",
  "term_id": "GO:0009636",
  "gene_symbol": "PON3",
  "gene_name": "Serum paraoxonase_lactonase 3",
  "gene": "UniProtKB:Q15166"
}